{
  "gene_name": "DNA polymerase subunit gamma-1",
  "gene": "UniProtKB:P54098",
  "term_label": "mitochondrion",
  "gene_symbol": "POLG",
  "term_id": "GO:0005739"
}